{
  "gene": "UniProtKB:Q9Y2A4",
  "gene_symbol": "ZNF443",
  "term_id": "GO:0000981",
  "gene_name": "Zinc finger protein 443",
  "term_label": "DNA-binding transcription factor activity, RNA polymerase II-specific"
}